{
  "gene": "UniProtKB:Q96RK0",
  "gene_name": "Protein capicua homolog",
  "term_label": "regulation of transcription by RNA polymerase II",
  "term_id": "GO:0006357",
  "gene_symbol": "CIC"
}